cellular response to glucose-phosphate stress [GO:0036448] (biological process) Relationships: is a type of cellular response to sugar-phosphate stress [GO:0036447] Definition: Any process that results in a change in state or activity of a cell (in terms of movement, secretion, enzyme production, gene expression, etc.) as a result of the accumulation of glucose-phosphate. References: PMID:17383224 Sources: GOC:am